D-arabitol catabolic process [GO:0051159] (biological process) Also known as: D-arabitol breakdown, D-arabitol catabolism, D-arabitol degradation Relationships: is a type of arabitol catabolic process [GO:0051157] Subtypes: D-arabitol catabolic process to D-xylulose 5-phosphate [GO:0019528] Sources: ISBN:0198506732 Definition: The chemical reactions and pathways resulting in the breakdown of D-arabitol, the pentitol derived from arabinose or lyxose by reduction of the aldehyde group. The D enantiomer is present in lichens and mushrooms.